negative regulation of estradiol secretion [GO:2000865] (biological process) Sources: GOC:sl Also known as: negative regulation of oestradiol secretion Definition: Any process that stops, prevents or reduces the frequency, rate or extent of estradiol secretion. Relationships: is a type of GO:2000832; is a type of regulation of estradiol secretion [GO:2000864]; negatively regulates estradiol secretion [GO:0035938]